{
  "gene": "UniProtKB:Q5SVS4",
  "gene_symbol": "SLC25A30",
  "term_label": "mitochondrial inner membrane",
  "gene_name": "Kidney mitochondrial carrier protein 1",
  "term_id": "GO:0005743"
}